{
  "gene_symbol": "PPP1R3A",
  "term_label": "regulation of glycogen biosynthetic process",
  "gene": "UniProtKB:Q16821",
  "gene_name": "Protein phosphatase 1 regulatory subunit 3A",
  "term_id": "GO:0005979"
}